{
  "term_id": "UNKNOWN:0001",
  "gene": "UniProtKB:Q04118",
  "gene_symbol": "PRB3",
  "gene_name": "Basic salivary proline-rich protein 3",
  "term_label": "Unknown molecular function"
}